{
  "term_id": "GO:0005200",
  "term_label": "structural constituent of cytoskeleton",
  "gene": "UniProtKB:Q8TDG2",
  "gene_name": "Actin-related protein T1",
  "gene_symbol": "ACTRT1"
}